{
  "term_label": "galactoside binding",
  "gene_symbol": "LGALS9",
  "gene": "UniProtKB:O00182",
  "gene_name": "Galectin-9",
  "term_id": "GO:0016936"
}